{
  "gene_symbol": "APOBEC3D",
  "gene": "UniProtKB:Q96AK3",
  "term_id": "GO:0016554",
  "term_label": "cytidine to uridine editing",
  "gene_name": "DNA dC-dU-editing enzyme APOBEC-3D"
}